{
  "term_label": "RSC-type complex",
  "gene_name": "Polycomb protein SUZ12",
  "gene_symbol": "SUZ12",
  "term_id": "GO:0016586",
  "gene": "UniProtKB:Q15022"
}